{
  "term_id": "GO:0006357",
  "gene_name": "Transcription factor SPT20 homolog",
  "gene": "UniProtKB:Q8NEM7",
  "term_label": "regulation of transcription by RNA polymerase II",
  "gene_symbol": "SUPT20H"
}